{
  "term_label": "voltage-gated calcium channel activity",
  "gene_symbol": "CACNG2",
  "gene": "UniProtKB:Q9Y698",
  "term_id": "GO:0005245",
  "gene_name": "Voltage-dependent calcium channel gamma-2 subunit"
}